{
  "gene_symbol": "STAP1",
  "gene_name": "Signal-transducing adaptor protein 1",
  "term_id": "UNKNOWN:0003",
  "term_label": "Unknown cellular component",
  "gene": "UniProtKB:Q9ULZ2"
}